antigen processing and presentation of exogenous peptide antigen [GO:0002478] (biological process) Relationships: is a type of antigen processing and presentation of exogenous antigen [GO:0019884]; is a type of antigen processing and presentation of peptide antigen [GO:0048002] Definition: The process in which an antigen-presenting cell expresses a peptide antigen of exogenous origin on its cell surface in association with an MHC protein complex. The peptide is typically a fragment of a larger exogenous protein which has been degraded within the cell. Also known as: exogenous peptide antigen processing and presentation Subtypes: antigen processing and presentation of exogenous peptide antigen via MHC class Ib [GO:0002477], antigen processing and presentation of exogenous peptide antigen via MHC class II [GO:0019886], antigen processing and presentation of exogenous peptide antigen via MHC class I [GO:0042590] Sources: GOC:add, ISBN:0781735149